{
  "term_id": "GO:0000731",
  "gene_name": "ATPase WRNIP1",
  "gene": "UniProtKB:Q96S55",
  "gene_symbol": "WRNIP1",
  "term_label": "DNA synthesis involved in DNA repair"
}